icosanoid receptor activity [GO:0004953] (molecular function) Relationships: is a type of G protein-coupled receptor activity [GO:0004930]; has part GO:0050542 Definition: Combining with an icosanoid to initiate a change in cell activity. Sources: GOC:dph Also known as: eicosanoid receptor activity Subtypes: prostanoid receptor activity [GO:0004954], leukotriene receptor activity [GO:0004974]